macrocin O-methyltransferase activity [GO:0030769] (molecular function) Definition: Catalysis of the reaction: S-adenosyl-L-methionine(1+) + macrocin = S-adenosyl-L-homocysteine + H+ + tylosin. Sources: EC:2.1.1.101, RHEA:17269 Also known as: S-adenosyl-L-methionine-macrocin O-methyltransferase activity, S-adenosyl-L-methionine:macrocin 3'''-O-methyltransferase activity, macrocin methyltransferase activity Relationships: is a type of GO:0008757